{
  "gene_symbol": "TMEM132C",
  "gene_name": "Transmembrane protein 132C",
  "term_id": "UNKNOWN:0002",
  "gene": "UniProtKB:Q8N3T6",
  "term_label": "Unknown biological process"
}